{
  "term_id": "GO:1990573",
  "gene": "UniProtKB:P50993",
  "gene_name": "Sodium_potassium-transporting ATPase subunit alpha-2",
  "gene_symbol": "ATP1A2",
  "term_label": "potassium ion import across plasma membrane"
}